{
  "term_id": "GO:0035435",
  "gene_name": "Glucose-6-phosphate exchanger SLC37A2",
  "term_label": "phosphate ion transmembrane transport",
  "gene_symbol": "SLC37A2",
  "gene": "UniProtKB:Q8TED4"
}